{
  "term_id": "GO:0071578",
  "gene_symbol": "SLC39A12",
  "gene_name": "Zinc transporter ZIP12",
  "term_label": "zinc ion import across plasma membrane",
  "gene": "UniProtKB:Q504Y0"
}